{
  "gene": "UniProtKB:Q6UXA7",
  "gene_name": "Uncharacterized protein C6orf15",
  "term_id": "GO:0031012",
  "term_label": "extracellular matrix",
  "gene_symbol": "C6orf15"
}